{
  "gene_name": "Homeobox and leucine zipper protein Homez",
  "term_label": "regulation of transcription by RNA polymerase II",
  "term_id": "GO:0006357",
  "gene_symbol": "HOMEZ",
  "gene": "UniProtKB:Q8IX15"
}